{
  "term_label": "Unknown biological process",
  "term_id": "UNKNOWN:0002",
  "gene_symbol": "IGHD3-9",
  "gene_name": "Immunoglobulin heavy diversity 3-9 (Fragment)",
  "gene": "UniProtKB:A0A0J9YW22"
}